{
  "gene_name": "UDP-glucuronosyltransferase 1A9",
  "gene": "UniProtKB:O60656",
  "term_id": "GO:0008210",
  "term_label": "estrogen metabolic process",
  "gene_symbol": "UGT1A9"
}